{
  "gene_symbol": "ACE2",
  "gene": "UniProtKB:Q9BYF1",
  "term_label": "metallopeptidase activity",
  "gene_name": "Angiotensin-converting enzyme 2",
  "term_id": "GO:0008237"
}